{
  "gene": "UniProtKB:Q96G75",
  "gene_symbol": "RMND5B",
  "term_label": "proteasome-mediated ubiquitin-dependent protein catabolic process",
  "term_id": "GO:0043161",
  "gene_name": "E3 ubiquitin-protein transferase RMND5B"
}